{
  "term_id": "GO:0005634",
  "gene": "UniProtKB:Q15940",
  "gene_name": "Putative zinc finger protein 726P1",
  "term_label": "nucleus",
  "gene_symbol": "ZNF726P1"
}